{
  "term_id": "GO:0034080",
  "term_label": "CENP-A containing chromatin assembly",
  "gene_symbol": "MIS18A",
  "gene_name": "Protein Mis18-alpha",
  "gene": "UniProtKB:Q9NYP9"
}